cardioblast anterior-lateral migration [GO:0003259] (biological process) Definition: The orderly movement of a cardioblast toward the head and laterally to form the heart field. A cardioblast is a cardiac precursor cell. It is a cell that has been committed to a cardiac fate, but will undergo more cell division rather than terminally differentiating. Relationships: is a type of cardioblast migration [GO:0003260] Sources: GOC:mtg_heart